{
  "gene": "UniProtKB:P36969",
  "gene_symbol": "GPX4",
  "term_label": "nucleus",
  "term_id": "GO:0005634",
  "gene_name": "Phospholipid hydroperoxide glutathione peroxidase"
}